{
  "gene": "UniProtKB:Q9UI46",
  "term_id": "GO:0045504",
  "gene_name": "Dynein axonemal intermediate chain 1",
  "gene_symbol": "DNAI1",
  "term_label": "dynein heavy chain binding"
}